{
  "gene": "UniProtKB:P58417",
  "term_id": "UNKNOWN:0003",
  "term_label": "Unknown cellular component",
  "gene_name": "Neurexophilin-1",
  "gene_symbol": "NXPH1"
}